corpus callosum development [GO:0022038] (biological process) Sources: GOC:cls, GOC:curators, GOC:dgh, GOC:dph, GOC:jid Relationships: is a type of anatomical structure development [GO:0048856]; is part of GO:0021537 Definition: The process whose specific outcome is the progression of the corpus callosum over time, from its formation to the mature structure. The corpus callosum is a thick bundle of nerve fibers comprising a commissural plate connecting the two cerebral hemispheres. It consists of contralateral axon projections that provide communication between the right and left cerebral hemispheres.